sorbitol-6-phosphatase activity [GO:0050286] (molecular function) Relationships: is a type of phosphatase activity [GO:0016791] Also known as: sorbitol-6-phosphate phosphatase activity, sorbitol-6-phosphate phosphohydrolase activity Sources: EC:3.1.3.50, RHEA:24580 Definition: Catalysis of the reaction: D-glucitol 6-phosphate + H2O = D-glucitol + phosphate.